{
  "gene_symbol": "RBPMS2",
  "term_label": "negative regulation of smooth muscle cell differentiation",
  "term_id": "GO:0051151",
  "gene": "UniProtKB:Q6ZRY4",
  "gene_name": "RNA-binding protein with multiple splicing 2"
}